IgA immunoglobulin complex, circulating [GO:0071746] (CC) Relationships: is a type of immunoglobulin complex, circulating [GO:0042571]; is a type of IgA immunoglobulin complex [GO:0071745] Subtypes: monomeric IgA immunoglobulin complex [GO:0071748], GO:0071749 Also known as: IgA antibody, IgA1 antibody, IgA2 antibody Note: Note that an IgA immunoglobulin complex has the function of antigen binding if a suitable antigen is available. References: PMID:16362985 Sources: GOC:add, ISBN:0781765196 Definition: A protein complex composed of two identical immunoglobulin heavy chains of an IgA isotype and two identical immunoglobulin light chains, held together by disulfide bonds, sometimes complexed with J chain or J chain and secretory component, and present in the extracellular space, in mucosal areas or other tissues, or circulating in the blood or lymph.